{
  "term_label": "heme biosynthetic process",
  "term_id": "GO:0006783",
  "gene_name": "Uroporphyrinogen decarboxylase",
  "gene": "UniProtKB:P06132",
  "gene_symbol": "UROD"
}